endomembrane system [GO:0012505] (cellular component) Definition: A collection of membranous structures involved in transport within the cell. The main components of the endomembrane system are endoplasmic reticulum, Golgi bodies, vesicles, cell membrane and nuclear envelope. Members of the endomembrane system pass materials through each other or though the use of vesicles. Sources: GOC:lh Relationships: is a type of GO:0110165; BFO_0000051 vacuole [GO:0005773]; has part GO:0005886